{
  "term_label": "Unknown cellular component",
  "term_id": "UNKNOWN:0003",
  "gene_symbol": "SAA1",
  "gene_name": "Serum amyloid A-1 protein",
  "gene": "UniProtKB:P0DJI8"
}